outer plaque of mitotic spindle pole body [GO:0061499] (cellular component) Sources: GOC:dph Relationships: is a type of outer plaque of spindle pole body [GO:0005824]; is part of mitotic spindle pole body [GO:0044732] Definition: One of three laminate structures that form the mitotic spindle pole body; the outer plaque is in the cytoplasm.